{
  "term_label": "phosphatidic acid transfer activity",
  "term_id": "GO:1990050",
  "gene": "UniProtKB:P55058",
  "gene_symbol": "PLTP",
  "gene_name": "Phospholipid transfer protein"
}